{
  "gene": "UniProtKB:Q9NZQ7",
  "gene_name": "Programmed cell death 1 ligand 1",
  "term_id": "GO:0071222",
  "term_label": "cellular response to lipopolysaccharide",
  "gene_symbol": "CD274"
}